sex determination, primary response to X:A ratio [GO:0007541] (biological process) Definition: The developmental process in which an organism interprets its X to autosomal chromosomal complement. Sources: GOC:isa_complete Relationships: is_a developmental process involved in reproduction [GO:0003006]; is part of primary sex determination, soma [GO:0007539]